{
  "term_label": "transforming growth factor beta receptor signaling pathway",
  "gene_name": "Zyxin",
  "gene_symbol": "ZYX",
  "term_id": "GO:0007179",
  "gene": "UniProtKB:Q15942"
}